{
  "term_label": "GTP binding",
  "term_id": "GO:0005525",
  "gene_symbol": "RAB4A",
  "gene_name": "Ras-related protein Rab-4A",
  "gene": "UniProtKB:P20338"
}